{
  "gene_symbol": "STRCP1",
  "term_id": "GO:0032426",
  "term_label": "stereocilium tip",
  "gene": "UniProtKB:A6NGW2",
  "gene_name": "Putative stereocilin-like protein"
}